{
  "term_label": "protein localization to actin cytoskeleton",
  "term_id": "GO:1903119",
  "gene": "UniProtKB:Q86V48",
  "gene_name": "Leucine zipper protein 1",
  "gene_symbol": "LUZP1"
}